{
  "gene_name": "Protein inturned",
  "term_label": "Unknown molecular function",
  "gene": "UniProtKB:Q9ULD6",
  "term_id": "UNKNOWN:0001",
  "gene_symbol": "INTU"
}